{
  "gene": "UniProtKB:Q53RY4",
  "gene_name": "Keratinocyte-associated protein 3",
  "term_id": "UNKNOWN:0001",
  "gene_symbol": "KRTCAP3",
  "term_label": "Unknown molecular function"
}